{
  "term_id": "GO:0003729",
  "gene_name": "Ras GTPase-activating protein-binding protein 2",
  "term_label": "mRNA binding",
  "gene": "UniProtKB:Q9UN86",
  "gene_symbol": "G3BP2"
}